{
  "gene_symbol": "DENND5A",
  "term_id": "GO:0031267",
  "gene": "UniProtKB:Q6IQ26",
  "gene_name": "DENN domain-containing protein 5A",
  "term_label": "small GTPase binding"
}